{
  "term_label": "actin filament organization",
  "gene_symbol": "MYO15A",
  "term_id": "GO:0007015",
  "gene_name": "Unconventional myosin-XV",
  "gene": "UniProtKB:Q9UKN7"
}